nuclear lamina [GO:0005652] (cellular component) Sources: ISBN:0198506732, ISBN:0716731363 Relationships: is a type of cellular anatomical structure [GO:0110165]; is part of nuclear envelope [GO:0005635]; is part of nuclear periphery [GO:0034399] Definition: The fibrous, electron-dense layer lying on the nucleoplasmic side of the inner membrane of a cell nucleus, composed of lamin filaments. The polypeptides of the lamina are thought to be concerned in the dissolution of the nuclear envelope and its re-formation during mitosis. The lamina is composed of lamin A and lamin C filaments cross-linked into an orthogonal lattice, which is attached via lamin B to the inner nuclear membrane through interactions with a lamin B receptor, an IFAP, in the membrane.